{
  "gene_symbol": "CD63",
  "term_id": "UNKNOWN:0001",
  "term_label": "Unknown molecular function",
  "gene": "UniProtKB:P08962",
  "gene_name": "CD63 antigen"
}